response to photoperiod, red light [GO:0009907] (BP) Sources: GOC:go_curators, GOC:mtg_far_red Relationships: is a type of GO:0009648; is a type of response to red light [GO:0010114] Definition: Any process that results in a change in state or activity of a cell or an organism (in terms of movement, secretion, enzyme production, gene expression, etc.) as a result of a red light photoperiod stimulus. Red light is electromagnetic radiation of wavelength of 580-700nm.